{
  "term_label": "cytoplasm",
  "gene_name": "Arf-GAP with dual PH domain-containing protein 2",
  "gene": "UniProtKB:Q9NPF8",
  "term_id": "GO:0005737",
  "gene_symbol": "ADAP2"
}